regulation of AMPA glutamate receptor clustering [GO:1904717] (biological process) Definition: Any process that modulates the frequency, rate or extent of AMPA glutamate receptor clustering. References: PMID:21558424 Sources: GOC:TermGenie, GOC:hjd, GO_REF:0000058 Also known as: regulation of AMPA receptor clustering, regulation of alpha-amino-3-hydroxy-5-methyl-4-isoxazole propionate selective glutamate receptor clustering Relationships: is a type of regulation of glutamate receptor clustering [GO:0106104]; regulates AMPA glutamate receptor clustering [GO:0097113] Subtypes: GO:1904718, positive regulation of AMPA glutamate receptor clustering [GO:1904719]